{
  "gene_name": "Potassium voltage-gated channel subfamily H member 3",
  "gene_symbol": "KCNH3",
  "term_label": "regulation of membrane potential",
  "gene": "UniProtKB:Q9ULD8",
  "term_id": "GO:0042391"
}